{
  "gene_symbol": "SPATA22",
  "term_label": "Unknown molecular function",
  "gene": "UniProtKB:Q8NHS9",
  "term_id": "UNKNOWN:0001",
  "gene_name": "Spermatogenesis-associated protein 22"
}